{
  "gene_name": "Interferon regulatory factor 5",
  "gene_symbol": "IRF5",
  "term_label": "DNA-binding transcription factor activity, RNA polymerase II-specific",
  "term_id": "GO:0000981",
  "gene": "UniProtKB:Q13568"
}